{
  "term_label": "RNA binding",
  "term_id": "GO:0003723",
  "gene_name": "Pescadillo homolog",
  "gene": "UniProtKB:O00541",
  "gene_symbol": "PES1"
}